{
  "term_id": "GO:0045944",
  "term_label": "positive regulation of transcription by RNA polymerase II",
  "gene_symbol": "HOXD4",
  "gene": "UniProtKB:P09016",
  "gene_name": "Homeobox protein Hox-D4"
}